{
  "gene_symbol": "SLC6A14",
  "term_label": "neutral, basic amino acid:sodium:chloride symporter activity",
  "gene": "UniProtKB:Q9UN76",
  "gene_name": "Sodium- and chloride-dependent neutral and basic amino acid transporter B(0+)",
  "term_id": "GO:0015374"
}